light absorption [GO:0016037] (biological process) Relationships: is a type of cellular process [GO:0009987]; is part of detection of light stimulus [GO:0009583] Sources: GOC:go_curators Also known as: absorption of light Definition: The reception of a photon by a cell. Subtypes: absorption of visible light [GO:0016038], GO:0016039